{
  "gene": "UniProtKB:Q6ZMC9",
  "term_label": "regulation of bone resorption",
  "gene_symbol": "SIGLEC15",
  "term_id": "GO:0045124",
  "gene_name": "Sialic acid-binding Ig-like lectin 15"
}